{
  "gene_symbol": "C1orf94",
  "gene_name": "Uncharacterized protein C1orf94",
  "term_label": "Unknown molecular function",
  "gene": "UniProtKB:Q6P1W5",
  "term_id": "UNKNOWN:0001"
}